{
  "gene": "UniProtKB:P51003",
  "term_label": "nucleus",
  "gene_symbol": "PAPOLA",
  "gene_name": "Poly(A) polymerase alpha",
  "term_id": "GO:0005634"
}